endocytosis involved in viral entry into host cell [GO:0075509] (biological process) Definition: Any endocytosis that is involved in the uptake of a virus into a host cell. Subtypes: receptor-mediated endocytosis of virus by host cell [GO:0019065], GO:0075510 Relationships: is a type of symbiont entry into host cell [GO:0046718] Also known as: viral penetration via endocytosis followed by endosome disruption, virus endocytosis by host, viral entry into host cell via endocytosis Sources: GOC:bf, GOC:jl, VZ:977